{
  "gene_symbol": "H2BC20P",
  "gene_name": "Putative histone H2B type 2-C",
  "term_id": "GO:0030527",
  "term_label": "structural constituent of chromatin",
  "gene": "UniProtKB:Q6DN03"
}